RNA-mediated DNA recombination [GO:0042152] (biological process) Definition: The reverse transcription of an RNA molecule followed by recombination between the resultant cDNA and its homologous chromosomal allele. References: PMID:8380627 Sources: GOC:jl Relationships: is_a GO:0006310